{
  "gene_symbol": "PRRG4",
  "term_id": "GO:0005615",
  "term_label": "extracellular space",
  "gene": "UniProtKB:Q9BZD6",
  "gene_name": "Transmembrane gamma-carboxyglutamic acid protein 4"
}